{
  "gene": "UniProtKB:O95049",
  "term_id": "GO:0005923",
  "gene_name": "Tight junction protein ZO-3",
  "term_label": "bicellular tight junction",
  "gene_symbol": "TJP3"
}